{
  "gene_symbol": "PAN3",
  "term_label": "poly(A) binding",
  "gene": "UniProtKB:Q58A45",
  "gene_name": "PAN2-PAN3 deadenylation complex subunit PAN3",
  "term_id": "GO:0008143"
}